alpha-heterochromatin [GO:0005723] (CC) Definition: A small, compact region of heterochromatin located in the middle of the polytene chromosome chromocenter, which undergoes little or no replication during polytenization. Relationships: is a type of GO:0005721; BFO_0000050 polytene chromosome chromocenter [GO:0005701] References: PMID:8878678